{
  "term_id": "GO:0045087",
  "gene": "UniProtKB:Q8IU54",
  "gene_name": "Interferon lambda-1",
  "gene_symbol": "IFNL1",
  "term_label": "innate immune response"
}